triplex DNA binding [GO:0045142] (molecular function) References: PMID:10681538 Definition: Binding to a DNA triple helix. The formation of triple helical DNA has been evoked in several cellular processes including transcription, replication, and recombination. Relationships: is a type of DNA binding [GO:0003677]